R3/R4 cell differentiation [GO:0048056] (BP) Definition: The process in which relatively unspecialized cells acquire the specialized features of R3 and R4 photoreceptors. An example of this process is found in Drosophila melanogaster. Sources: GOC:jid Relationships: is a type of compound eye photoreceptor cell differentiation [GO:0001751]